positive regulation of antral ovarian follicle growth [GO:2000388] (biological process) Definition: Any process that activates or increases the frequency, rate or extent of antral ovarian follicle growth. Relationships: is a type of GO:0048639; is_a positive regulation of reproductive process [GO:2000243]; is a type of regulation of antral ovarian follicle growth [GO:2000387]; positively regulates antral ovarian follicle growth [GO:0001547] Sources: GOC:obol